cell outer membrane [GO:0009279] (cellular component) Sources: GOC:md, GOC:mtg_sensu, ISBN:0135712254 Also known as: outer membrane of cell Subtypes: mycolate outer membrane [GO:0036407] Note: To annotate the plasma (cytoplasmic) membrane, see instead GO:0005886. Relationships: is a type of outer membrane [GO:0019867]; is part of external encapsulating structure [GO:0030312]; is part of cell envelope [GO:0030313] Definition: A lipid bilayer that forms the outermost membrane of the cell envelope; enriched in polysaccharide and protein; the outer leaflet of the membrane contains specific lipopolysaccharide structures.